{
  "term_id": "UNKNOWN:0001",
  "gene_name": "Pleckstrin homology-like domain family A member 2",
  "term_label": "Unknown molecular function",
  "gene_symbol": "PHLDA2",
  "gene": "UniProtKB:Q53GA4"
}